D-allose 6-phosphate isomerase activity [GO:0008786] (molecular function) Sources: RHEA:28430 Also known as: allose 6-phosphate isomerase activity Relationships: is a type of intramolecular oxidoreductase activity, interconverting aldoses and ketoses [GO:0016861] Definition: Catalysis of the reaction: D-allose-6-phosphate = D-allulose-6-phosphate.